{
  "term_label": "Unknown biological process",
  "term_id": "UNKNOWN:0002",
  "gene": "UniProtKB:P13725",
  "gene_name": "Oncostatin-M",
  "gene_symbol": "OSM"
}